{
  "gene_symbol": "ARL14EP",
  "gene": "UniProtKB:Q8N8R7",
  "gene_name": "ARL14 effector protein",
  "term_label": "Unknown cellular component",
  "term_id": "UNKNOWN:0003"
}